{
  "term_id": "GO:0001731",
  "term_label": "formation of translation preinitiation complex",
  "gene_name": "Eukaryotic translation initiation factor 2 subunit 3B",
  "gene": "UniProtKB:Q2VIR3",
  "gene_symbol": "EIF2S3B"
}